{
  "term_id": "GO:0004842",
  "gene_name": "ORC ubiquitin ligase 1",
  "term_label": "ubiquitin-protein transferase activity",
  "gene": "UniProtKB:Q5W0B1",
  "gene_symbol": "OBI1"
}